{
  "gene": "UniProtKB:Q9NPD7",
  "term_label": "Unknown molecular function",
  "term_id": "UNKNOWN:0001",
  "gene_name": "Neuritin",
  "gene_symbol": "NRN1"
}